{
  "gene_name": "Transcription initiation protein SPT3 homolog",
  "gene": "UniProtKB:O75486",
  "term_label": "Unknown cellular component",
  "term_id": "UNKNOWN:0003",
  "gene_symbol": "SUPT3H"
}